ATP-dependent H2AZ histone chaperone activity [GO:0140849] (molecular function) Relationships: is a type of GO:0140674 Also known as: ATP-dependent H2A.Z histone chaperone activity, H2AZ histone exchange activity Definition: A histone chaperone that mediates the exchange of histone H2A-H2B dimer and histone H2AZ-H2B dimers in a nucleosome, driven by ATP hydrolysis. Some chaperones insert H2AZ-H2B dimers and remove H2A-H2B, while others do the opposite. References: PMID:21241891, PMID:23580526, PMID:30309918 Note: Drosophila H2AV corresponds to histone H2AZ.